{
  "gene_symbol": "MTUS2",
  "gene_name": "Microtubule-associated tumor suppressor candidate 2",
  "term_label": "cytoplasm",
  "term_id": "GO:0005737",
  "gene": "UniProtKB:Q5JR59"
}